{
  "gene": "UniProtKB:P17213",
  "term_id": "GO:0043031",
  "gene_symbol": "BPI",
  "gene_name": "Bactericidal permeability-increasing protein",
  "term_label": "negative regulation of macrophage activation"
}